phosphoenolpyruvate carboxylase activity [GO:0008964] (molecular function) Definition: Catalysis of the reaction: phosphate + oxaloacetate = phosphoenolpyruvate + HCO3-. Also known as: PEP carboxylase activity, PEPC, PEPCase activity, phosphate:oxaloacetate carboxy-lyase (adding phosphate; phosphoenolpyruvate-forming), phosphate:oxaloacetate carboxy-lyase (phosphorylating), phosphoenolpyruvic carboxylase activity, phosphopyruvate (phosphate) carboxylase activity Sources: EC:4.1.1.31 Relationships: is a type of phosphoenolpyruvate carboxykinase activity [GO:0004611]